labyrinthine layer formation [GO:0060714] (biological process) Definition: The developmental process pertaining to the initial formation of the labyrinthine layer of the placenta. Sources: GOC:dph Relationships: is a type of anatomical structure formation involved in morphogenesis [GO:0048646]; is part of labyrinthine layer morphogenesis [GO:0060713]